{
  "term_id": "GO:0000715",
  "gene_name": "DNA repair protein complementing XP-A cells",
  "gene": "UniProtKB:P23025",
  "gene_symbol": "XPA",
  "term_label": "nucleotide-excision repair, DNA damage recognition"
}